anagen [GO:0042640] (biological process) Definition: The growth phase of the hair cycle. Lasts, for example, about 3 to 6 years for human scalp hair. References: PMID:12230507 Also known as: hair growth Note: Note that this term should not be used for direct annotation. If you are trying to make an annotation to x phase, it is likely that the correct annotation is 'regulation of x/y phase transition' or to a process which occurs during the reported phase. To capture the phase when a specific location or process is observed, the phase term can be used in an annotation extension (PMID:24885854) applied to a cellular component term (with the relation exists_during) or a biological process term (with the relation happens_during). Relationships: is a type of hair cycle phase [GO:0044851]; BFO_0000050 hair follicle maturation [GO:0048820] Regulation: regulated by regulation of timing of anagen [GO:0051884]; positively regulated by positive regulation of timing of anagen [GO:0051885]; negatively regulated by GO:0051886